myelination of lateral line nerve axons [GO:0048897] (biological process) Definition: The formation of compact myelin sheaths around the axons of a lateral line nerve. References: PMID:12112375 Relationships: is a type of myelination [GO:0042552]; is part of GO:0048938 Subtypes: myelination of anterior lateral line nerve axons [GO:0048914], myelination of posterior lateral line nerve axons [GO:0048932]